{
  "gene_symbol": "CDC45",
  "term_id": "GO:0031261",
  "term_label": "DNA replication preinitiation complex",
  "gene": "UniProtKB:O75419",
  "gene_name": "Cell division control protein 45 homolog"
}